growth cone lamellipodium [GO:1990761] (cellular component) Definition: A thin sheetlike process extended by the leading edge of an axonal or dendritic growth cone; contains a dense meshwork of actin filaments. References: PMID:25598228 Sources: GOC:dos Relationships: is a type of GO:0030027; is a type of GO:0043005; is part of growth cone [GO:0030426]